{
  "gene_symbol": "CC2D1B",
  "term_label": "RNA polymerase II cis-regulatory region sequence-specific DNA binding",
  "term_id": "GO:0000978",
  "gene": "UniProtKB:Q5T0F9",
  "gene_name": "Coiled-coil and C2 domain-containing protein 1B"
}